{
  "term_label": "negative regulation of canonical Wnt signaling pathway",
  "gene": "UniProtKB:Q9NQB0",
  "gene_name": "Transcription factor 7-like 2",
  "term_id": "GO:0090090",
  "gene_symbol": "TCF7L2"
}